{
  "gene": "UniProtKB:O75752",
  "gene_name": "UDP-GalNAc:beta-1,3-N-acetylgalactosaminyltransferase 1",
  "term_id": "GO:0008499",
  "gene_symbol": "B3GALNT1",
  "term_label": "N-acetyl-beta-D-glucosaminide beta-(1,3)-galactosyltransferase activity"
}